{
  "gene_symbol": "ZER1",
  "term_id": "UNKNOWN:0002",
  "term_label": "Unknown biological process",
  "gene_name": "Protein zer-1 homolog",
  "gene": "UniProtKB:Q7Z7L7"
}